{
  "gene": "UniProtKB:O60729",
  "gene_name": "Dual specificity protein phosphatase CDC14B",
  "gene_symbol": "CDC14B",
  "term_id": "GO:0005737",
  "term_label": "cytoplasm"
}